{
  "gene": "UniProtKB:P29803",
  "gene_symbol": "PDHA2",
  "term_label": "pyruvate dehydrogenase complex",
  "gene_name": "Pyruvate dehydrogenase E1 component subunit alpha, testis-specific form, mitochondrial",
  "term_id": "GO:0045254"
}